{
  "gene_name": "T cell receptor beta variable 10-3",
  "gene_symbol": "TRBV10-3",
  "term_id": "GO:0005886",
  "gene": "UniProtKB:A0A0K0K1G6",
  "term_label": "plasma membrane"
}